all-trans retinoic acid 18-hydroxylase activity [GO:0062183] (molecular function) Definition: Catalysis of the reaction: all-trans-retinoate + O2 + reduced [NADPH--hemoprotein reductase] = all-trans-18-hydroxyretinoate + H+ + H2O + oxidized [NADPH--hemoprotein reductase]. References: PMID:22020119 Sources: RHEA:55856 Relationships: is a type of monooxygenase activity [GO:0004497]